{
  "gene": "UniProtKB:P51685",
  "gene_symbol": "CCR8",
  "term_label": "cell chemotaxis",
  "gene_name": "C-C chemokine receptor type 8",
  "term_id": "GO:0060326"
}